monoatomic ion antiporter activity involved in regulation of presynaptic membrane potential [GO:0099520] (molecular function) Relationships: is a type of antiporter activity [GO:0015297]; occurs in presynaptic membrane [GO:0042734] Sources: GOC:dos Definition: Any ion antiporter activity, occurring in the presynaptic membrane, that is involved in regulation of presynaptic membrane potential. Also known as: ion antiporter activity involved in regulation of pre-synaptic membrane potential, ion antiporter activity involved in regulation of presynaptic membrane potential